{
  "gene_symbol": "RDH5",
  "term_label": "retinoid metabolic process",
  "gene_name": "Retinol dehydrogenase 5",
  "gene": "UniProtKB:Q92781",
  "term_id": "GO:0001523"
}